cell-substrate junction disassembly [GO:0120180] (biological process) References: PMID:25490267 Sources: GOC:aruk, GOC:bc Relationships: is a type of cell-substrate junction organization [GO:0150115]; is a type of cell junction disassembly [GO:0150146] Definition: The disaggregation of a cell-substrate junction into its constituent components. Subtypes: focal adhesion disassembly [GO:0120181]